{
  "gene_name": "Poly(rC)-binding protein 1",
  "gene_symbol": "PCBP1",
  "term_label": "single-stranded DNA binding",
  "term_id": "GO:0003697",
  "gene": "UniProtKB:Q15365"
}